{
  "term_label": "phospholipid efflux",
  "gene": "UniProtKB:Q9H2V7",
  "gene_name": "Protein spinster homolog 1",
  "gene_symbol": "SPNS1",
  "term_id": "GO:0033700"
}